{
  "gene_symbol": "ACSM2A",
  "gene_name": "Acyl-coenzyme A synthetase ACSM2A, mitochondrial",
  "term_label": "fatty acid biosynthetic process",
  "term_id": "GO:0006633",
  "gene": "UniProtKB:Q08AH3"
}